{
  "gene": "UniProtKB:O00203",
  "term_id": "GO:0016192",
  "term_label": "vesicle-mediated transport",
  "gene_symbol": "AP3B1",
  "gene_name": "AP-3 complex subunit beta-1"
}